{
  "gene": "UniProtKB:Q2NL67",
  "term_id": "GO:0030968",
  "gene_name": "Protein mono-ADP-ribosyltransferase PARP6",
  "gene_symbol": "PARP6",
  "term_label": "endoplasmic reticulum unfolded protein response"
}